modulation by host of viral glycoprotein metabolic process [GO:0044870] (biological process) Sources: GOC:jl Relationships: is a type of host-mediated perturbation of viral process [GO:0044788]; RO_0002211 glycoprotein metabolic process [GO:0009100] Definition: A process in which a host organism modulates the frequency, rate or extent of viral glycoprotein metabolic process. Subtypes: GO:0044871